{
  "gene_symbol": "RHEX",
  "term_label": "Unknown molecular function",
  "term_id": "UNKNOWN:0001",
  "gene": "UniProtKB:Q6ZWK4",
  "gene_name": "Regulator of hemoglobinization and erythroid cell expansion protein"
}